wing disc development [GO:0035220] (biological process) Definition: Progression of the wing disc over time, from its initial formation through to its metamorphosis to form adult structures including the wing hinge, wing blade and pleura. Subtypes: determination of wing disc primordium [GO:0035294] Relationships: is a type of imaginal disc development [GO:0007444] Sources: GOC:bf, ISBN:0879694238